{
  "gene_symbol": "TOR1A",
  "gene": "UniProtKB:O14656",
  "gene_name": "Torsin-1A",
  "term_id": "GO:0005635",
  "term_label": "nuclear envelope"
}